{
  "term_id": "UNKNOWN:0003",
  "gene_symbol": "TMEM208",
  "term_label": "Unknown cellular component",
  "gene": "UniProtKB:Q9BTX3",
  "gene_name": "Transmembrane protein 208"
}